exo-(1,4)-alpha-D-glucan lyase activity [GO:0047457] (molecular function) Also known as: alpha-1,4-glucan lyase activity, (1->4)-alpha-D-glucan exo-4-lyase (1,5-anhydro-D-fructose-forming), alpha-(1->4)-glucan 1,5-anhydro-D-fructose eliminase activity, alpha-1,4-glucan 1,5-anhydro-D-fructose eliminase activity, alpha-1,4-glucan exo-lyase activity, exo-(1->4)-alpha-D-glucan lyase activity, exo-alpha-1,4-glucan lyase activity Sources: EC:4.2.2.13, MetaCyc:4.2.2.13-RXN Definition: Catalysis of the reaction: linear alpha-D-glucan = 1,5-anhydro-D-fructose + beta-D-glucose. Relationships: is a type of GO:0016837